{
  "gene": "UniProtKB:Q96GY3",
  "term_label": "Myb complex",
  "gene_symbol": "LIN37",
  "term_id": "GO:0031523",
  "gene_name": "Protein lin-37 homolog"
}